dynactin complex [GO:0005869] (CC) Definition: A 20S multiprotein assembly of total mass about 1.2 MDa that activates dynein-based activity in vivo. A large structural component of the complex is an actin-like 40 nm filament composed of actin-related protein, to which other components attach. Sources: ISBN:0198506732 Relationships: is a type of microtubule associated complex [GO:0005875]; is part of GO:0015629